{
  "term_label": "maternal aggressive behavior",
  "term_id": "GO:0002125",
  "gene_symbol": "OXT",
  "gene": "UniProtKB:P01178",
  "gene_name": "Oxytocin-neurophysin 1"
}